ureter smooth muscle contraction [GO:0014849] (biological process) Relationships: is a type of GO:0014821; is a type of urinary tract smooth muscle contraction [GO:0014848] Definition: A process in which force is generated within smooth muscle tissue, resulting in a change in muscle geometry. This process occurs in the ureter. Force generation involves a chemo-mechanical energy conversion step that is carried out by the actin/myosin complex activity, which generates force through ATP hydrolysis. The ureter is one of a pair of thick-walled tubes that transports urine from the kidney pelvis to the urinary bladder. Sources: GOC:mtg_muscle, MA:0000378 Subtypes: GO:0072105